{
  "term_id": "UNKNOWN:0001",
  "gene_symbol": "FAM174B",
  "gene_name": "Membrane protein FAM174B",
  "term_label": "Unknown molecular function",
  "gene": "UniProtKB:Q3ZCQ3"
}